regulation of fibronectin-dependent thymocyte migration [GO:2000413] (biological process) Definition: Any process that modulates the frequency, rate or extent of fibronectin-dependent thymocyte migration. Relationships: is a type of regulation of thymocyte migration [GO:2000410]; regulates fibronectin-dependent thymocyte migration [GO:0072681] Sources: GOC:mah Subtypes: negative regulation of fibronectin-dependent thymocyte migration [GO:2000414], GO:2000415 Also known as: regulation of fibronectin-dependent thymic lymphocyte migration, regulation of fibronectin-dependent immature T cell migration, regulation of fibronectin-dependent immature T lymphocyte migration, regulation of fibronectin-dependent immature T-cell migration, regulation of fibronectin-dependent immature T-lymphocyte migration